{
  "term_id": "GO:0005829",
  "gene_name": "Glyoxylate reductase_hydroxypyruvate reductase",
  "gene": "UniProtKB:Q9UBQ7",
  "gene_symbol": "GRHPR",
  "term_label": "cytosol"
}